{
  "gene_name": "Janus kinase and microtubule-interacting protein 1",
  "term_id": "UNKNOWN:0002",
  "gene": "UniProtKB:Q96N16",
  "gene_symbol": "JAKMIP1",
  "term_label": "Unknown biological process"
}